{
  "term_label": "Unknown molecular function",
  "gene_name": "Torsin-1A-interacting protein 1",
  "gene_symbol": "TOR1AIP1",
  "term_id": "UNKNOWN:0001",
  "gene": "UniProtKB:Q5JTV8"
}